{
  "term_id": "UNKNOWN:0001",
  "gene": "UniProtKB:Q8N0U2",
  "term_label": "Unknown molecular function",
  "gene_name": "Transmembrane protein 61",
  "gene_symbol": "TMEM61"
}